RNA polymerase III assembly [GO:1990115] (biological process) Definition: The aggregation, arrangement and bonding together of a set of components to form the eukaryotic RNA polymerase III complex. References: PMID:23459708 Sources: GOC:rb Also known as: DNA-directed RNA polymerase III complex assembly, RNA Polymerase III complex assembly Relationships: is_a protein-containing complex assembly [GO:0065003]